{
  "gene": "UniProtKB:O95343",
  "gene_name": "Homeobox protein SIX3",
  "term_id": "GO:0001654",
  "term_label": "eye development",
  "gene_symbol": "SIX3"
}